{
  "term_label": "flavin adenine dinucleotide binding",
  "gene_name": "NADPH-dependent diflavin oxidoreductase 1",
  "term_id": "GO:0050660",
  "gene": "UniProtKB:Q9UHB4",
  "gene_symbol": "NDOR1"
}